{
  "gene_name": "Cytoplasmic polyadenylation element-binding protein 3",
  "term_id": "GO:0007616",
  "term_label": "long-term memory",
  "gene": "UniProtKB:Q8NE35",
  "gene_symbol": "CPEB3"
}